regulation of pronephros size [GO:0035565] (biological process) Also known as: regulation of pronephric kidney size Definition: Any process that modulates the size of a pronephric kidney. Relationships: is a type of regulation of kidney size [GO:0035564]; is part of GO:0072114 Sources: GOC:bf